{
  "gene": "UniProtKB:P30519",
  "gene_name": "Heme oxygenase 2",
  "term_label": "heme oxidation",
  "gene_symbol": "HMOX2",
  "term_id": "GO:0006788"
}